columbamine oxidase activity [GO:0050455] (molecular function) Sources: RHEA:23564 Relationships: is a type of oxidoreductase activity, acting on X-H and Y-H to form an X-Y bond, with oxygen as acceptor [GO:0046993] Definition: Catalysis of the reaction: 2 columbamine + O2 = 2 berberine + 2 H2O. Also known as: berberine synthase activity, columbamine:oxygen oxidoreductase (cyclizing)